{
  "term_id": "GO:0045236",
  "term_label": "CXCR chemokine receptor binding",
  "gene_name": "Stromal cell-derived factor 1",
  "gene_symbol": "CXCL12",
  "gene": "UniProtKB:P48061"
}